{
  "gene_symbol": "CREB3",
  "gene": "UniProtKB:O43889",
  "term_label": "DNA-binding transcription factor activity, RNA polymerase II-specific",
  "term_id": "GO:0000981",
  "gene_name": "Cyclic AMP-responsive element-binding protein 3"
}